{
  "gene": "UniProtKB:Q99928",
  "term_label": "benzodiazepine receptor activity",
  "term_id": "GO:0008503",
  "gene_symbol": "GABRG3",
  "gene_name": "Gamma-aminobutyric acid receptor subunit gamma-3"
}